{
  "gene_symbol": "RDH13",
  "gene": "UniProtKB:Q8NBN7",
  "term_id": "GO:0010842",
  "gene_name": "Retinol dehydrogenase 13",
  "term_label": "retina layer formation"
}